{
  "gene_name": "Cysteine protease ATG4C",
  "term_id": "GO:0034727",
  "term_label": "piecemeal microautophagy of the nucleus",
  "gene_symbol": "ATG4C",
  "gene": "UniProtKB:Q96DT6"
}